{
  "gene_symbol": "PIGZ",
  "gene": "UniProtKB:Q86VD9",
  "gene_name": "GPI mannosyltransferase 4",
  "term_label": "alpha-1,2-mannosyltransferase activity",
  "term_id": "GO:0000026"
}